{
  "term_id": "GO:0005886",
  "gene": "UniProtKB:O00161",
  "term_label": "plasma membrane",
  "gene_name": "Synaptosomal-associated protein 23",
  "gene_symbol": "SNAP23"
}